{
  "gene_name": "Ubiquitin-protein ligase E3A",
  "term_id": "GO:0061630",
  "term_label": "ubiquitin protein ligase activity",
  "gene": "UniProtKB:Q05086",
  "gene_symbol": "UBE3A"
}